axon initial segment [GO:0043194] (cellular component) Also known as: initial segment Relationships: is a type of GO:0110165; is part of main axon [GO:0044304] Definition: Portion of the axon proximal to the neuronal cell body, at the level of the axon hillock. The action potentials that propagate along the axon are generated at the level of this initial segment. References: PMID:1754851, PMID:21551097 Sources: GOC:nln, GOC:sl